{
  "gene_symbol": "CIAO2A",
  "gene": "UniProtKB:Q9H5X1",
  "term_label": "Unknown molecular function",
  "gene_name": "Cytosolic iron-sulfur assembly component 2A",
  "term_id": "UNKNOWN:0001"
}